{
  "term_id": "GO:0006623",
  "gene_symbol": "VPS13A",
  "term_label": "protein targeting to vacuole",
  "gene_name": "Intermembrane lipid transfer protein VPS13A",
  "gene": "UniProtKB:Q96RL7"
}